{
  "term_label": "Unknown molecular function",
  "term_id": "UNKNOWN:0001",
  "gene_name": "tRNA (guanine-N(7)-)-methyltransferase non-catalytic subunit WDR4",
  "gene": "UniProtKB:P57081",
  "gene_symbol": "WDR4"
}